{
  "gene_name": "M-phase phosphoprotein 8",
  "gene_symbol": "MPHOSPH8",
  "gene": "UniProtKB:Q99549",
  "term_id": "GO:0062072",
  "term_label": "histone H3K9me2/3 reader activity"
}